{
  "gene_name": "Copine-8",
  "term_id": "GO:0005886",
  "term_label": "plasma membrane",
  "gene_symbol": "CPNE8",
  "gene": "UniProtKB:Q86YQ8"
}